positive regulation of NAD(P)H oxidase activity [GO:0033864] (biological process) Sources: GOC:mah Definition: Any process that activates or increases the activity of the enzyme NAD(P)H oxidase. Also known as: up regulation of NAD(P)H oxidase activity, up-regulation of NAD(P)H oxidase activity, upregulation of NAD(P)H oxidase activity, activation of NAD(P)H oxidase activity, stimulation of NAD(P)H oxidase activity Relationships: is a type of GO:0051353; positively regulates NAD(P)H oxidase H2O2-forming activity [GO:0016174]